{
  "term_id": "UNKNOWN:0002",
  "gene_name": "Leucine-rich repeat and calponin homology domain-containing protein 2",
  "gene_symbol": "LRCH2",
  "gene": "UniProtKB:Q5VUJ6",
  "term_label": "Unknown biological process"
}